{
  "gene_name": "Cofilin-1",
  "gene": "UniProtKB:P23528",
  "gene_symbol": "CFL1",
  "term_label": "actin cytoskeleton",
  "term_id": "GO:0015629"
}